coenzyme A diphosphatase activity [GO:0010945] (molecular function) References: PMID:10922370, PMID:16185196 Also known as: CoA diphosphatase activity, CoA pyrophosphatase activity, coenzyme A pyrophosphatase activity Definition: Catalysis of the reaction: an acyl-coenzyme A or its derivatives + H2O = adenosine 3',5'-bisphosphate + an acyl-4'-phosphopantetheine + 2 H+. This reaction can also use coenzyme A as a substrate. Relationships: is_a GO:0016462